oxidoreductase activity, acting on hydrogen as donor [GO:0016695] (molecular function) Definition: Catalysis of an oxidation-reduction (redox) reaction in which hydrogen acts as an electron donor. Also known as: oxidoreductase activity, acting on hydrogen as donor, other acceptors Subtypes: oxidoreductase activity, acting on hydrogen as donor, NAD or NADP as acceptor [GO:0016696], oxidoreductase activity, acting on hydrogen as donor, cytochrome as acceptor [GO:0016697], oxidoreductase activity, acting on hydrogen as donor, iron-sulfur protein as acceptor [GO:0016699], hydrogenase (acceptor) activity [GO:0033748], oxidoreductase activity, acting on hydrogen as donor, with a quinone or similar compound as acceptor [GO:0046994], oxidoreductase activity, acting on hydrogen as donor, with other known acceptors [GO:0046995] Sources: GOC:jl Relationships: is a type of oxidoreductase activity [GO:0016491]